{
  "gene": "UniProtKB:Q6PI77",
  "term_id": "GO:0005829",
  "gene_name": "G protein-coupled receptor associated sorting protein 3",
  "gene_symbol": "GPRASP3",
  "term_label": "cytosol"
}